{
  "term_id": "GO:0000145",
  "term_label": "exocyst",
  "gene_name": "Exocyst complex component 6B",
  "gene": "UniProtKB:Q9Y2D4",
  "gene_symbol": "EXOC6B"
}